{
  "gene_symbol": "GOLGA6L26",
  "gene_name": "Golgin subfamily A member 6-like protein 26",
  "term_label": "Unknown molecular function",
  "term_id": "UNKNOWN:0001",
  "gene": "UniProtKB:P0DX02"
}